lipid translocation [GO:0034204] (biological process) Subtypes: glycolipid translocation [GO:0034203], phospholipid translocation [GO:0045332], sphingolipid translocation [GO:0099039] Sources: GOC:mah Definition: The translocation, or flipping, of lipid molecules from one monolayer of a membrane bilayer to the opposite monolayer. Also known as: intramembrane lipid transfer Relationships: is a type of lipid transport [GO:0006869]; is a type of regulation of membrane lipid distribution [GO:0097035]